regulation of memory T cell activation [GO:2000567] (biological process) Sources: GOC:obol Subtypes: positive regulation of memory T cell activation [GO:2000568] Definition: Any process that modulates the frequency, rate or extent of memory T cell activation. Relationships: is_a regulation of T cell activation [GO:0050863]; RO_0002211 memory T cell activation [GO:0035709]